negative regulation of vascular associated smooth muscle cell differentiation [GO:1905064] (biological process) Relationships: is a type of GO:0051151; is a type of regulation of vascular associated smooth muscle cell differentiation [GO:1905063]; negatively regulates GO:0035886 References: PMID:19088079 Sources: GOC:BHF, GOC:BHF_miRNA, GOC:TermGenie, GOC:rph, GO_REF:0000058 Definition: Any process that stops, prevents or reduces the frequency, rate or extent of vascular smooth muscle cell differentiation. Subtypes: negative regulation of aortic smooth muscle cell differentiation [GO:1904830], GO:1905931, negative regulation of cardiac vascular smooth muscle cell differentiation [GO:2000723] Also known as: down regulation of VSMC differentiation, down regulation of vascular associated smooth muscle cell differentiation, down regulation of vascular smooth muscle cell differentiation, down-regulation of VSMC differentiation, down-regulation of vascular associated smooth muscle cell differentiation, down-regulation of vascular smooth muscle cell differentiation, downregulation of VSMC differentiation, downregulation of vascular associated smooth muscle cell differentiation, downregulation of vascular smooth muscle cell differentiation, negative regulation of VSMC differentiation, negative regulation of vascular smooth muscle cell differentiation, inhibition of VSMC differentiation, inhibition of vascular associated smooth muscle cell differentiation, inhibition of vascular smooth muscle cell differentiation